{
  "term_id": "GO:0042567",
  "gene_symbol": "IGFALS",
  "gene_name": "Insulin-like growth factor-binding protein complex acid labile subunit",
  "term_label": "insulin-like growth factor ternary complex",
  "gene": "UniProtKB:P35858"
}